{
  "gene_name": "Cytochrome P450 7B1",
  "term_id": "GO:0042632",
  "term_label": "cholesterol homeostasis",
  "gene": "UniProtKB:O75881",
  "gene_symbol": "CYP7B1"
}